{
  "gene": "UniProtKB:Q9Y426",
  "gene_name": "C2 domain-containing protein 2",
  "gene_symbol": "C2CD2",
  "term_label": "Unknown cellular component",
  "term_id": "UNKNOWN:0003"
}